2-oxoglutarate metabolic process [GO:0006103] (biological process) Definition: The chemical reactions and pathways involving oxoglutarate, the dianion of 2-oxoglutaric acid. It is a key constituent of the TCA cycle and a key intermediate in amino-acid metabolism. Relationships: is a type of GO:0043648 Also known as: 2-ketoglutarate metabolic process, 2-ketoglutarate metabolism, 2-oxoglutarate metabolism, alpha-ketoglutarate metabolic process, alpha-ketoglutarate metabolism, alpha-oxoglutarate metabolic process, alpha-oxoglutarate metabolism Subtypes: proline catabolic process to 2-oxoglutarate [GO:0019495], L-histidine catabolic process to 2-oxoglutarate [GO:0019558], L-arabinose catabolic process to 2-oxoglutarate [GO:0019570], mixed acid fermentation [GO:0019664], acetyl-CoA assimilation pathway [GO:0019681], 2-oxoglutarate decarboxylation to succinyl-CoA [GO:0120551] Sources: ISBN:0198506732